entry of viral genome into host nucleus via docking of viral capsid to the nuclear pore complex and injection of viral genome [GO:0075507] (biological process) Definition: Viral penetration into the host nucleus where the where a viral capsid docks on the cytoplasmic side of the nuclear pore complex (NPC) and ejects the viral genome through the pore into the nucleoplasm. Note: This mechanism is used by viruses such as Herpesvirales whose capsid is too large to enter the nuclear pore complex (NPC) pore. Relationships: is a type of viral penetration into host nucleus [GO:0075732] References: PMID:22929056 Sources: VZ:989